{
  "gene_symbol": "NCF1B",
  "gene": "UniProtKB:A6NI72",
  "term_id": "GO:0005737",
  "term_label": "cytoplasm",
  "gene_name": "Putative neutrophil cytosol factor 1B"
}